{
  "term_label": "nucleosomal DNA binding",
  "gene_symbol": "H3-3B",
  "gene_name": "Histone H3.3",
  "gene": "UniProtKB:P84243",
  "term_id": "GO:0031492"
}